negative regulation of citrulline biosynthetic process [GO:1903249] (biological process) Definition: Any process that stops, prevents or reduces the frequency, rate or extent of citrulline biosynthetic process. References: PMID:19278978 Sources: GOC:BHF, GOC:TermGenie, GOC:rl, GO_REF:0000058 Also known as: down regulation of citrulline anabolism, down regulation of citrulline biosynthesis, down regulation of citrulline biosynthetic process, down regulation of citrulline formation, down regulation of citrulline synthesis, down-regulation of citrulline anabolism, down-regulation of citrulline biosynthesis, down-regulation of citrulline biosynthetic process, down-regulation of citrulline formation, down-regulation of citrulline synthesis, downregulation of citrulline anabolism, downregulation of citrulline biosynthesis, downregulation of citrulline biosynthetic process, downregulation of citrulline formation, downregulation of citrulline synthesis, negative regulation of citrulline anabolism, negative regulation of citrulline biosynthesis, negative regulation of citrulline formation, negative regulation of citrulline synthesis, inhibition of citrulline anabolism, inhibition of citrulline biosynthesis, inhibition of citrulline biosynthetic process, inhibition of citrulline formation, inhibition of citrulline synthesis Relationships: is a type of negative regulation of small molecule metabolic process [GO:0062014]; is a type of regulation of citrulline biosynthetic process [GO:1903248]; is a type of negative regulation of amino acid biosynthetic process [GO:2000283]; negatively regulates citrulline biosynthetic process [GO:0019240]